{
  "term_label": "positive regulation of cytokine-mediated signaling pathway",
  "term_id": "GO:0001961",
  "gene_symbol": "CD74",
  "gene": "UniProtKB:P04233",
  "gene_name": "HLA class II histocompatibility antigen gamma chain"
}